{
  "gene": "UniProtKB:P54253",
  "gene_symbol": "ATXN1",
  "term_label": "nucleus",
  "gene_name": "Ataxin-1",
  "term_id": "GO:0005634"
}